histone lactyltransferase (CoA-dependent) activity [GO:0120301] (molecular function) Relationships: is a type of peptide lactyltransferase (CoA-dependent) activity [GO:0120300]; is a type of GO:0140993 Definition: Catalysis of the reaction: (L-lysyl-[histone] + lactoyl-CoA = CoA + H+ + N(6)-lactoyl-L-lysyl-[histone]. Also known as: histone lactyltransferase activity, histone lactyltransferase (CoA dependent) activity, histone lactyltransferase activity (CoA dependent) References: PMID:31645732 Sources: GOC:sp